alpha9-beta1 integrin-ADAM2 complex [GO:0071053] (cellular component) Relationships: is a type of plasma membrane protein complex [GO:0098797] Also known as: ITGA9-ITGB1-ADAM2 complex Definition: A protein complex that consists of an alpha9-beta1 integrin complex bound to the transmembrane metallopeptidase ADAM2. References: PMID:11882657